{
  "gene_symbol": "H3Y1",
  "term_label": "nucleus",
  "gene_name": "Histone H3.Y",
  "term_id": "GO:0005634",
  "gene": "UniProtKB:P0DPK2"
}